cell wall disassembly involved in floral organ abscission [GO:0060870] (biological process) Relationships: is a type of cell wall modification involved in abscission [GO:0009830]; is part of floral organ abscission [GO:0010227] Sources: GOC:dph, GOC:sdb_2009, GOC:tb Definition: A cellular process that results in the breakdown of the cell wall that contributes to the process of floral organ abscission.